{
  "gene_name": "Ras-responsive element-binding protein 1",
  "gene_symbol": "RREB1",
  "term_id": "GO:0001228",
  "gene": "UniProtKB:Q92766",
  "term_label": "DNA-binding transcription activator activity, RNA polymerase II-specific"
}